positive regulation of plasma kallikrein-kinin cascade [GO:0002550] (biological process) Definition: Any process that activates or increases the frequency, rate, or extent of the plasma kallikrein-kinin cascade. Sources: GOC:add Also known as: up regulation of plasma kallikrein-kinin cascade, up-regulation of plasma kallikrein-kinin cascade, upregulation of plasma kallikrein-kinin cascade, activation of plasma kallikrein-kinin cascade, stimulation of plasma kallikrein-kinin cascade Relationships: is a type of positive regulation of kinin cascade [GO:0002258]; is a type of regulation of plasma kallikrein-kinin cascade [GO:0002529]; positively regulates plasma kallikrein-kinin cascade [GO:0002353]